{
  "gene_symbol": "ABHD12B",
  "term_label": "endoplasmic reticulum membrane",
  "gene": "UniProtKB:Q7Z5M8",
  "gene_name": "Protein ABHD12B",
  "term_id": "GO:0005789"
}